{
  "gene_name": "Replication factor C subunit 4",
  "term_id": "GO:0005634",
  "term_label": "nucleus",
  "gene": "UniProtKB:P35249",
  "gene_symbol": "RFC4"
}